{
  "gene_symbol": "KCNAB2",
  "gene_name": "Voltage-gated potassium channel subunit beta-2",
  "term_label": "alcohol dehydrogenase (NADP+) activity",
  "term_id": "GO:0008106",
  "gene": "UniProtKB:Q13303"
}